{
  "gene_name": "Keratin, type I cytoskeletal 26",
  "term_label": "epithelial cell differentiation",
  "gene": "UniProtKB:Q7Z3Y9",
  "gene_symbol": "KRT26",
  "term_id": "GO:0030855"
}